{
  "gene_name": "Olfactory receptor 4P4",
  "gene_symbol": "OR4P4",
  "term_label": "olfactory receptor activity",
  "term_id": "GO:0004984",
  "gene": "UniProtKB:Q8NGL7"
}